mitochondrial transport [GO:0006839] (biological process) Definition: Transport of substances into, out of or within a mitochondrion. Sources: GOC:ai Relationships: is a type of intracellular transport [GO:0046907] Subtypes: mitochondrion to lysosome vesicle-mediated transport [GO:0099074], GO:1990542